{
  "gene_name": "BTB_POZ domain-containing protein 18",
  "term_label": "piRNA transcription",
  "term_id": "GO:0140541",
  "gene": "UniProtKB:B2RXH4",
  "gene_symbol": "BTBD18"
}